extracellular core region of desmosome [GO:0090635] (CC) Also known as: desmoglea Definition: The desmosomal part containing the desmosomal cadherins, desmogleins and desmocollins, that establish contact and adhere to neighboring cells in a Ca2+-dependent manner. References: PMID:20066089 Relationships: is a type of cellular anatomical structure [GO:0110165]; is part of GO:0030057